methionine adenosyltransferase complex [GO:0048269] (cellular component) Relationships: is a type of GO:0140535; is_a transferase complex [GO:1990234] Also known as: MAT complex Definition: A multimeric enzyme complex composed of variable numbers of catalytic alpha subunits, and noncatalytic beta subunits. The beta subunits are believed to have a regulatory function. The enzyme complex catalyzes the synthesis of S-adenosylmethionine (AdoMet), which is the major methyl group donor, participating in the methylation of proteins, DNA, RNA, phospholipids, and other small molecules. References: PMID:10644686, PMID:25075345 Sources: GOC:jid